{
  "gene_symbol": "UTP3",
  "gene": "UniProtKB:Q9NQZ2",
  "term_id": "GO:0005730",
  "term_label": "nucleolus",
  "gene_name": "Something about silencing protein 10"
}